{
  "gene_symbol": "TEKT1",
  "term_id": "UNKNOWN:0001",
  "gene_name": "Tektin-1",
  "gene": "UniProtKB:Q969V4",
  "term_label": "Unknown molecular function"
}